{
  "gene_name": "Tumor protein p73",
  "term_label": "chromatin",
  "gene": "UniProtKB:O15350",
  "term_id": "GO:0000785",
  "gene_symbol": "TP73"
}